{
  "gene_name": "Tripartite motif-containing protein 46",
  "term_id": "GO:0001578",
  "gene": "UniProtKB:Q7Z4K8",
  "term_label": "microtubule bundle formation",
  "gene_symbol": "TRIM46"
}